{
  "term_label": "RNA polymerase II cis-regulatory region sequence-specific DNA binding",
  "gene": "UniProtKB:Q92766",
  "gene_symbol": "RREB1",
  "gene_name": "Ras-responsive element-binding protein 1",
  "term_id": "GO:0000978"
}